{
  "term_label": "structural constituent of skin epidermis",
  "gene_symbol": "KRT34",
  "gene_name": "Keratin, type I cuticular Ha4",
  "term_id": "GO:0030280",
  "gene": "UniProtKB:O76011"
}